negative regulation of type II interferon-mediated signaling pathway [GO:0060336] (biological process) Definition: Any process that decreases the rate, frequency or extent of an interferon-gamma-mediated signaling pathway. Sources: GOC:dph Also known as: negative regulation of interferon-gamma-mediated signaling pathway, negative regulation of type II IFN-mediated signaling pathway, negative regulation of immune interferon-mediated signaling pathway, negative regulation of interferon-gamma-mediated signalling pathway, negative regulation of gamma-interferon-mediated signaling pathway Relationships: is a type of negative regulation of cytokine-mediated signaling pathway [GO:0001960]; is a type of negative regulation of response to type II interferon [GO:0060331]; is a type of regulation of type II interferon-mediated signaling pathway [GO:0060334]; negatively regulates type II interferon-mediated signaling pathway [GO:0060333]